{
  "term_label": "Unknown molecular function",
  "gene_symbol": "SMARCAL1",
  "gene_name": "SWI_SNF-related matrix-associated actin-dependent regulator of chromatin subfamily A-like protein 1",
  "term_id": "UNKNOWN:0001",
  "gene": "UniProtKB:Q9NZC9"
}